{
  "gene_symbol": "SYNE4",
  "term_id": "GO:0005640",
  "gene_name": "Nesprin-4",
  "gene": "UniProtKB:Q8N205",
  "term_label": "nuclear outer membrane"
}